{
  "gene_name": "Terminal uridylyltransferase 4",
  "term_id": "GO:0031123",
  "term_label": "RNA 3'-end processing",
  "gene": "UniProtKB:Q5TAX3",
  "gene_symbol": "TUT4"
}